{
  "term_id": "UNKNOWN:0001",
  "term_label": "Unknown molecular function",
  "gene_symbol": "MRPS27",
  "gene": "UniProtKB:Q92552",
  "gene_name": "Small ribosomal subunit protein mS27"
}